triglyceride mobilization [GO:0006642] (biological process) References: PMID:11943743, PMID:15713625 Sources: GOC:mah Also known as: triacylglycerol mobilization Relationships: is a type of triglyceride metabolic process [GO:0006641] Definition: The release of triglycerides, any triester of glycerol, from storage within cells or tissues, making them available for metabolism.